{
  "gene": "UniProtKB:Q9P2H3",
  "gene_name": "Intraflagellar transport protein 80 homolog",
  "gene_symbol": "IFT80",
  "term_label": "intraciliary transport particle B",
  "term_id": "GO:0030992"
}